{
  "term_label": "mitochondrial NAD transmembrane transport",
  "term_id": "GO:1990549",
  "gene_name": "Mitochondrial nicotinamide adenine dinucleotide transporter SLC25A51",
  "gene": "UniProtKB:Q9H1U9",
  "gene_symbol": "SLC25A51"
}